{
  "term_label": "MAP kinase phosphatase activity",
  "gene_symbol": "DUSP3",
  "gene": "UniProtKB:P51452",
  "term_id": "GO:0033549",
  "gene_name": "Dual specificity protein phosphatase 3"
}